{
  "gene": "UniProtKB:Q9ULF5",
  "term_label": "intracellular monoatomic cation homeostasis",
  "term_id": "GO:0030003",
  "gene_name": "Zinc transporter ZIP10",
  "gene_symbol": "SLC39A10"
}